{
  "gene_symbol": "PRPS1L1",
  "term_label": "ribose phosphate diphosphokinase complex",
  "gene_name": "Ribose-phosphate pyrophosphokinase 3",
  "gene": "UniProtKB:P21108",
  "term_id": "GO:0002189"
}